stereocilia tip link [GO:0002140] (cellular component) References: PMID:1108787 Relationships: is_a stereocilia coupling link [GO:0002139] Definition: A stereocilia link that is formed by a fine filament running more or less vertically upward from the tip of each shorter stereocilium to attach at a higher point on its adjacent taller neighbor. Tilting the bundle puts tension on the filaments, which pull on mechanically gated ion channels in the membrane of the stereocilia.